{
  "term_label": "protein import into nucleus",
  "term_id": "GO:0006606",
  "gene_symbol": "TNPO3",
  "gene_name": "Transportin-3",
  "gene": "UniProtKB:Q9Y5L0"
}